{
  "gene_name": "Annexin A1",
  "term_id": "GO:0012506",
  "gene_symbol": "ANXA1",
  "term_label": "vesicle membrane",
  "gene": "UniProtKB:P04083"
}